{
  "term_label": "cell chemotaxis",
  "gene_symbol": "DEFB110",
  "gene": "UniProtKB:Q30KQ9",
  "term_id": "GO:0060326",
  "gene_name": "Beta-defensin 110"
}